{
  "gene_symbol": "DPEP2",
  "term_id": "GO:0005886",
  "gene": "UniProtKB:Q9H4A9",
  "term_label": "plasma membrane",
  "gene_name": "Dipeptidase 2"
}